protein localization to heterochromatin [GO:0097355] (biological process) Also known as: protein localisation to heterochromatin Relationships: is a type of protein localization to chromatin [GO:0071168] Sources: GOC:mah Definition: Any process in which a protein is transported to, or maintained at, a part of a chromosome that is organized into heterochromatin. Subtypes: CLRC complex localization to heterochromatin [GO:0044382], protein localization to pericentric heterochromatin [GO:1902682], protein localization to mating-type region heterochromatin [GO:1903212], protein localization to subtelomeric heterochromatin [GO:1903213]